{
  "term_id": "GO:0005125",
  "gene": "UniProtKB:P01588",
  "term_label": "cytokine activity",
  "gene_symbol": "EPO",
  "gene_name": "Erythropoietin"
}